{
  "term_label": "endoplasmic reticulum membrane",
  "gene": "UniProtKB:O00401",
  "term_id": "GO:0005789",
  "gene_name": "Actin nucleation-promoting factor WASL",
  "gene_symbol": "WASL"
}